fatty-acyl-CoA binding [GO:0000062] (molecular function) Sources: GOC:jl, GOC:krc, ISBN:0198506732 Definition: Binding to a fatty-acyl-CoA, any derivative of coenzyme A in which the sulfhydryl group is in thiolester linkage with a fatty acyl group. Also known as: fatty-acyl binding, fatty-acyl-coenzyme A binding Relationships: is a type of acyl-CoA binding [GO:0120227]; is a type of fatty acid derivative binding [GO:1901567] Subtypes: long-chain fatty acyl-CoA binding [GO:0036042]